{
  "term_label": "protein ubiquitination",
  "gene": "UniProtKB:Q9UII4",
  "term_id": "GO:0016567",
  "gene_name": "E3 ISG15--protein ligase HERC5",
  "gene_symbol": "HERC5"
}